{
  "gene_name": "Paraneoplastic antigen Ma6E",
  "term_label": "Unknown biological process",
  "gene_symbol": "PNMA6E",
  "gene": "UniProtKB:A0A0J9YXQ4",
  "term_id": "UNKNOWN:0002"
}